{
  "term_label": "cytokine activity",
  "term_id": "GO:0005125",
  "gene": "UniProtKB:O95760",
  "gene_symbol": "IL33",
  "gene_name": "Interleukin-33"
}